{
  "term_label": "snRNA binding",
  "gene": "UniProtKB:Q16560",
  "term_id": "GO:0017069",
  "gene_symbol": "SNRNP35",
  "gene_name": "U11_U12 small nuclear ribonucleoprotein 35 kDa protein"
}